{
  "term_label": "Unknown molecular function",
  "gene": "UniProtKB:Q86UD5",
  "gene_name": "Sodium_hydrogen exchanger 9B2",
  "gene_symbol": "SLC9B2",
  "term_id": "UNKNOWN:0001"
}